{
  "gene_name": "Periostin",
  "gene": "UniProtKB:Q15063",
  "term_id": "GO:0030198",
  "term_label": "extracellular matrix organization",
  "gene_symbol": "POSTN"
}